(-)-pinoresinol catabolic process [GO:1902123] (BP) Definition: The chemical reactions and pathways resulting in the breakdown of (-)-pinoresinol. Also known as: (-)-pinoresinol breakdown, (-)-pinoresinol catabolism, (-)-pinoresinol degradation References: PMID:15949826, PMID:9872995 Sources: GOC:TermGenie Relationships: is a type of phenol-containing compound catabolic process [GO:0019336]; is_a GO:0046273; is a type of ether catabolic process [GO:1901502]; is a type of (-)-pinoresinol metabolic process [GO:1901598]